response to iron(III) ion [GO:0010041] (biological process) Subtypes: cellular response to iron(III) ion [GO:0071283] Relationships: is a type of response to iron ion [GO:0010039] Definition: Any process that results in a change in state or activity of a cell or an organism (in terms of movement, secretion, enzyme production, gene expression, etc.) as a result of an iron(III) ion stimulus. Also known as: response to iron(III) Sources: GOC:sm